{
  "term_label": "transmembrane transporter complex",
  "gene_name": "Zinc-activated ligand-gated ion channel",
  "term_id": "GO:1902495",
  "gene": "UniProtKB:Q401N2",
  "gene_symbol": "ZACN"
}